UDP-sulfoquinovose:DAG sulfoquinovosyltransferase activity [GO:0046510] (molecular function) Also known as: sulfolipid synthase, UDP-sulphoquinovose:DAG sulphoquinovosyltransferase activity Definition: Catalysis of the reaction: UDP-sulfoquinovose + 1,2-diacylglycerol = sulfoquinovosyldiacylglycerol + UDP. Sources: MetaCyc:RXN-1224 Relationships: is a type of UDP-glycosyltransferase activity [GO:0008194]; is a type of hexosyltransferase activity [GO:0016758]